{
  "term_label": "N,N-dimethylaniline monooxygenase activity",
  "gene": "UniProtKB:Q99518",
  "term_id": "GO:0004499",
  "gene_symbol": "FMO2",
  "gene_name": "Flavin-containing monooxygenase 2"
}